{
  "gene_symbol": "PERM1",
  "gene": "UniProtKB:Q5SV97",
  "gene_name": "PGC-1 and ERR-induced regulator in muscle protein 1",
  "term_id": "UNKNOWN:0001",
  "term_label": "Unknown molecular function"
}